{
  "term_label": "regulation of transcription by RNA polymerase II",
  "gene_symbol": "NPAS3",
  "term_id": "GO:0006357",
  "gene": "UniProtKB:Q8IXF0",
  "gene_name": "Neuronal PAS domain-containing protein 3"
}